response to chemokine [GO:1990868] (biological process) Definition: Any process that results in a change in state or activity of a cell or an organism (in terms of movement, secretion, enzyme production, gene expression, etc.) as a result of a chemokine stimulus. References: PMID:11113082 Relationships: is a type of GO:0034097 Subtypes: cellular response to chemokine [GO:1990869]